positive regulation of adaptive immune response [GO:0002821] (biological process) Relationships: is a type of regulation of adaptive immune response [GO:0002819]; is a type of positive regulation of immune response [GO:0050778]; positively regulates adaptive immune response [GO:0002250] Also known as: up regulation of adaptive immune response, up-regulation of adaptive immune response, upregulation of adaptive immune response, activation of adaptive immune response, stimulation of adaptive immune response Sources: GOC:add Subtypes: positive regulation of adaptive immune response based on somatic recombination of immune receptors built from immunoglobulin superfamily domains [GO:0002824], positive regulation of adaptive immune memory response [GO:1905676], positive regulation of adaptive immune effector response [GO:1905679] Definition: Any process that activates or increases the frequency, rate, or extent of an adaptive immune response.